{
  "gene": "UniProtKB:Q92563",
  "gene_name": "Testican-2",
  "term_label": "extracellular space",
  "term_id": "GO:0005615",
  "gene_symbol": "SPOCK2"
}